cell gliding [GO:0071976] (biological process) Definition: Cell motility that results in the smooth movement of a cell along a solid surface. References: PMID:18461074 Subtypes: adventurous gliding motility [GO:0030982], cell surface adhesin-mediated gliding motility [GO:0071980] Also known as: cell gliding motility Relationships: is a type of cell motility [GO:0048870]